oxamate carbamoyltransferase activity [GO:0050205] (molecular function) Also known as: carbamoyl-phosphate:oxamate carbamoyltransferase activity, oxamic transcarbamylase activity Sources: EC:2.1.3.5, RHEA:22984 Definition: Catalysis of the reaction: carbamoyl phosphate + oxamate = oxalurate + phosphate. Relationships: is a type of carboxyl- or carbamoyltransferase activity [GO:0016743]